{
  "term_id": "GO:0006955",
  "gene": "UniProtKB:P51684",
  "gene_symbol": "CCR6",
  "gene_name": "C-C chemokine receptor type 6",
  "term_label": "immune response"
}